regulation of translational initiation in response to stress [GO:0043558] (biological process) Sources: GOC:jl Also known as: regulation of translation initiation in response to stress Relationships: is a type of regulation of translational initiation [GO:0006446]; is a type of GO:0043555 Subtypes: GO:0010998, negative regulation of translation in response to oxidative stress [GO:0032938], regulation of translation initiation in response to endoplasmic reticulum stress [GO:0036491], regulation of translational initiation by eIF2 alpha dephosphorylation [GO:0036496], regulation of translational initiation in response to osmotic stress [GO:0043561], regulation of translational initiation in response to starvation [GO:0071262], regulation of cytoplasmic translational initiation in response to stress [GO:1990611] Definition: Any process that modulates the frequency, rate or extent of translation initiation, as a result of a stimulus indicating the organism is under stress.